{
  "term_label": "heart development",
  "gene_symbol": "TGFB2",
  "gene": "UniProtKB:P61812",
  "gene_name": "Transforming growth factor beta-2 proprotein",
  "term_id": "GO:0007507"
}